{
  "gene_symbol": "PLK3",
  "gene": "UniProtKB:Q9H4B4",
  "term_id": "GO:0007052",
  "term_label": "mitotic spindle organization",
  "gene_name": "Serine_threonine-protein kinase PLK3"
}